{
  "gene": "UniProtKB:O15254",
  "term_label": "pristanoyl-CoA oxidase activity",
  "term_id": "GO:0016402",
  "gene_symbol": "ACOX3",
  "gene_name": "Peroxisomal acyl-coenzyme A oxidase 3"
}